positive regulation of focal adhesion disassembly [GO:0120183] (biological process) Definition: Any process that activates or increases the frequency, rate or extent of disaggregation of a focal adhesion into its constituent components. Relationships: is a type of regulation of focal adhesion disassembly [GO:0120182]; is a type of positive regulation of cell-substrate junction organization [GO:0150117]; RO_0002213 GO:0120181 References: PMID:25490267